{
  "gene_name": "Gamma-interferon-inducible protein 16",
  "gene": "UniProtKB:Q16666",
  "term_id": "GO:0002218",
  "term_label": "activation of innate immune response",
  "gene_symbol": "IFI16"
}